proteasome storage granule disassembly [GO:1902907] (biological process) References: PMID:23690178 Sources: GOC:TermGenie, GOC:di, GO_REF:0000079 Relationships: is_a organelle disassembly [GO:1903008] Also known as: PSG disassembly Definition: The disaggregation of a proteasome storage granule into its constituent components.